positive regulation of cytokinin-activated signaling pathway [GO:0080038] (biological process) Definition: Any process that activates or increases the frequency, rate or extent of cytokinin signaling. Sources: GOC:dhl Also known as: positive regulation of cytokinin mediated signalling, positive regulation of cytokinin mediated signaling pathway Relationships: is a type of GO:0009967; is a type of regulation of cytokinin-activated signaling pathway [GO:0080036]; positively regulates cytokinin-activated signaling pathway [GO:0009736]